{
  "gene": "UniProtKB:P01571",
  "gene_symbol": "IFNA17",
  "gene_name": "Interferon alpha-17",
  "term_label": "response to exogenous dsRNA",
  "term_id": "GO:0043330"
}